phosphatidylserine exposure on blood platelet [GO:0097045] (biological process) Relationships: is a type of GO:0017121; is a type of positive regulation of blood coagulation [GO:0030194] Definition: A phospholipid scrambling process that results in the appearance of phosphatidylserine on the surface of activated blood platelets, and triggers the clotting system. References: PMID:21107324 Sources: GOC:bf, GOC:lf, GOC:pr